{
  "term_label": "Unknown cellular component",
  "term_id": "UNKNOWN:0003",
  "gene": "UniProtKB:Q02930",
  "gene_symbol": "CREB5",
  "gene_name": "Cyclic AMP-responsive element-binding protein 5"
}